{
  "term_label": "benzodiazepine receptor activity",
  "gene_symbol": "GABRA6",
  "gene": "UniProtKB:Q16445",
  "gene_name": "Gamma-aminobutyric acid receptor subunit alpha-6",
  "term_id": "GO:0008503"
}